{
  "term_label": "protoheme IX farnesyltransferase activity",
  "gene_name": "Protoheme IX farnesyltransferase, mitochondrial",
  "term_id": "GO:0008495",
  "gene_symbol": "COX10",
  "gene": "UniProtKB:Q12887"
}